{
  "term_id": "GO:0000723",
  "gene": "UniProtKB:Q70YC5",
  "gene_symbol": "ZNF365",
  "gene_name": "Protein ZNF365",
  "term_label": "telomere maintenance"
}